{
  "term_label": "Unknown molecular function",
  "gene_name": "Peptidase inhibitor 16",
  "gene_symbol": "PI16",
  "gene": "UniProtKB:Q6UXB8",
  "term_id": "UNKNOWN:0001"
}